{
  "term_id": "GO:0005815",
  "term_label": "microtubule organizing center",
  "gene_symbol": "KIAA0753",
  "gene": "UniProtKB:Q2KHM9",
  "gene_name": "Protein moonraker"
}